{
  "gene": "UniProtKB:Q8TE68",
  "term_id": "GO:0035023",
  "term_label": "regulation of Rho protein signal transduction",
  "gene_symbol": "EPS8L1",
  "gene_name": "Epidermal growth factor receptor kinase substrate 8-like protein 1"
}